{
  "gene": "UniProtKB:Q6ZQY2",
  "gene_name": "Leucine-rich repeat-containing protein 74B",
  "term_label": "Unknown biological process",
  "term_id": "UNKNOWN:0002",
  "gene_symbol": "LRRC74B"
}